Atg12 activating enzyme activity [GO:0019778] (molecular function) Sources: GOC:mah Also known as: APG12 activating enzyme activity Definition: Catalysis of the activation of the small ubiquitin-related modifier APG12, through the formation of an ATP-dependent high-energy thiolester bond. Relationships: is a type of ubiquitin-like modifier activating enzyme activity [GO:0008641]